AF-2 domain binding [GO:0050682] (molecular function) Relationships: is a type of protein domain specific binding [GO:0019904] References: PMID:9682036 Definition: Binding to an AF-2 protein domain, a highly conserved ligand-dependent transactivation domain which is essential for receptor-mediated transcriptional activation.